somatic diversification of T cell receptor genes by N region addition [GO:0002571] (biological process) Definition: The addition of variable numbers of random nucleotides by terminal deoxytransferase in the N regions of T cell receptor genes. N regions are found at the V-D, D-D, V-J, and D-J recombinational junctions, depending on the T cell receptor gene. Sources: GOC:add, ISBN:0781735149 Also known as: somatic diversification of TCR genes by N region addition Relationships: is a type of somatic diversification of T cell receptor genes [GO:0002568]; is a type of somatic diversification of immune receptors by N region addition [GO:0002569]; is part of somatic recombination of T cell receptor gene segments [GO:0002681]